{
  "term_id": "GO:0060326",
  "gene_symbol": "RHOG",
  "gene_name": "Rho-related GTP-binding protein RhoG",
  "term_label": "cell chemotaxis",
  "gene": "UniProtKB:P84095"
}